toll-like receptor 5 signaling pathway [GO:0034146] (biological process) References: PMID:16551253, PMID:17328678 Sources: GOC:add Definition: The series of molecular signals initiated by a ligand binding to toll-like receptor 5. Regulation: regulated by regulation of toll-like receptor 5 signaling pathway [GO:0034147]; negatively regulated by negative regulation of toll-like receptor 5 signaling pathway [GO:0034148]; positively regulated by positive regulation of toll-like receptor 5 signaling pathway [GO:0034149] Relationships: is a type of GO:0140895 Also known as: TLR5 signaling pathway, toll-like receptor 5 signalling pathway